{
  "gene": "UniProtKB:Q02224",
  "gene_symbol": "CENPE",
  "term_label": "microtubule-based movement",
  "term_id": "GO:0007018",
  "gene_name": "Centromere-associated protein E"
}